{
  "gene_symbol": "DNAAF4",
  "term_id": "GO:0036158",
  "gene": "UniProtKB:Q8WXU2",
  "term_label": "outer dynein arm assembly",
  "gene_name": "Dynein axonemal assembly factor 4"
}